{
  "term_label": "1-phosphatidylinositol 4-kinase activity",
  "gene": "UniProtKB:Q9UBF8",
  "term_id": "GO:0004430",
  "gene_name": "Phosphatidylinositol 4-kinase beta",
  "gene_symbol": "PI4KB"
}